{
  "term_label": "regulation of synaptic vesicle exocytosis",
  "gene_symbol": "SYT8",
  "term_id": "GO:2000300",
  "gene_name": "Synaptotagmin-8",
  "gene": "UniProtKB:Q8NBV8"
}